{
  "term_id": "GO:0005634",
  "gene_symbol": "TLK1",
  "gene_name": "Serine_threonine-protein kinase tousled-like 1",
  "gene": "UniProtKB:Q9UKI8",
  "term_label": "nucleus"
}